{
  "term_label": "heterochromatin",
  "gene_symbol": "MECP2",
  "term_id": "GO:0000792",
  "gene_name": "Methyl-CpG-binding protein 2",
  "gene": "UniProtKB:P51608"
}